{
  "gene_symbol": "ZNF408",
  "term_id": "GO:0000978",
  "gene": "UniProtKB:Q9H9D4",
  "gene_name": "Zinc finger protein 408",
  "term_label": "RNA polymerase II cis-regulatory region sequence-specific DNA binding"
}